liver trabecula formation [GO:0060344] (biological process) Also known as: liver trabeculation, liver trabecula biogenesis Sources: GOC:dph Relationships: is a type of trabecula formation [GO:0060343]; is part of liver development [GO:0001889] Definition: The process of creating a trabecula in the liver. A trabecula is a tissue element in the form of a small beam, strut or rod.